{
  "gene": "UniProtKB:A8MPY1",
  "term_id": "GO:0005254",
  "gene_symbol": "GABRR3",
  "gene_name": "Gamma-aminobutyric acid receptor subunit rho-3",
  "term_label": "chloride channel activity"
}